{
  "gene_name": "Tyrosine-protein kinase receptor UFO",
  "gene": "UniProtKB:P30530",
  "term_id": "GO:0007169",
  "term_label": "cell surface receptor protein tyrosine kinase signaling pathway",
  "gene_symbol": "AXL"
}